{
  "term_id": "GO:0004674",
  "term_label": "protein serine/threonine kinase activity",
  "gene_symbol": "TSSK3",
  "gene_name": "Testis-specific serine_threonine-protein kinase 3",
  "gene": "UniProtKB:Q96PN8"
}